{
  "term_id": "GO:0050911",
  "gene_symbol": "OR10A6",
  "gene": "UniProtKB:Q8NH74",
  "term_label": "detection of chemical stimulus involved in sensory perception of smell",
  "gene_name": "Olfactory receptor 10A6"
}